{
  "gene": "UniProtKB:Q9NWW0",
  "gene_symbol": "HCFC1R1",
  "term_label": "Unknown biological process",
  "term_id": "UNKNOWN:0002",
  "gene_name": "Host cell factor C1 regulator 1"
}